{
  "gene_name": "Bactericidal permeability-increasing protein",
  "gene_symbol": "BPI",
  "term_label": "innate immune response",
  "gene": "UniProtKB:P17213",
  "term_id": "GO:0045087"
}